{
  "term_id": "GO:0005886",
  "gene_name": "Mu-type opioid receptor",
  "gene": "UniProtKB:P35372",
  "term_label": "plasma membrane",
  "gene_symbol": "OPRM1"
}